{
  "term_id": "UNKNOWN:0002",
  "term_label": "Unknown biological process",
  "gene": "UniProtKB:F2Z398",
  "gene_name": "LMO7 downstream neighbor protein",
  "gene_symbol": "LMO7DN"
}